{
  "term_label": "Unknown molecular function",
  "gene": "UniProtKB:Q5T319",
  "gene_symbol": "FAM182B",
  "term_id": "UNKNOWN:0001",
  "gene_name": "Protein FAM182B"
}